vomilenine glucosyltransferase activity [GO:0050506] (molecular function) Sources: EC:2.4.1.219, RHEA:19385 Definition: Catalysis of the reaction: UDP-D-glucose + vomilenine = H+ + raucaffricine + UDP. Relationships: is a type of UDP-glucosyltransferase activity [GO:0035251] Also known as: UDP-glucose:vomilenine 21-O-beta-D-glucosyltransferase activity, UDPG:vomilenine 21-beta-D-glucosyltransferase activity, UDPG:vomilenine 21beta-D-glucosyltransferase activity, vomilenine-glucosyltransferase activity